negative regulation of monoatomic ion transport [GO:0043271] (biological process) Subtypes: negative regulation of sodium ion transport [GO:0010766], GO:0014063, GO:0034757, negative regulation of monoatomic ion transmembrane transport [GO:0034766], negative regulation of potassium ion transport [GO:0043267], negative regulation of calcium ion transport [GO:0051926], negative regulation of zinc ion transport [GO:0071582], GO:1903792 Also known as: negative regulation of ion transport, down regulation of ion transport, down-regulation of ion transport, downregulation of ion transport, inhibition of ion transport Relationships: is_a regulation of monoatomic ion transport [GO:0043269]; is a type of GO:0051051; negatively regulates monoatomic ion transport [GO:0006811] Sources: GOC:jl Definition: Any process that stops, prevents, or reduces the frequency, rate or extent of the directed movement of charged atoms or small charged molecules into, out of or within a cell, or between cells, by means of some agent such as a transporter or pore.